{
  "term_label": "Unknown biological process",
  "gene_symbol": "Q6ZQY7",
  "gene": "UniProtKB:Q6ZQY7",
  "term_id": "UNKNOWN:0002",
  "gene_name": "Putative uncharacterized protein FLJ46792"
}